{
  "gene": "UniProtKB:A8MPP1",
  "gene_symbol": "DDX11L8",
  "term_id": "GO:0005634",
  "gene_name": "Putative ATP-dependent RNA helicase DDX11-like protein 8",
  "term_label": "nucleus"
}